{
  "gene_symbol": "LMNB1",
  "gene_name": "Lamin-B1",
  "term_id": "GO:0031507",
  "term_label": "heterochromatin formation",
  "gene": "UniProtKB:P20700"
}